{
  "gene_symbol": "OR10H5",
  "gene_name": "Olfactory receptor 10H5",
  "term_id": "GO:0050911",
  "gene": "UniProtKB:Q8NGA6",
  "term_label": "detection of chemical stimulus involved in sensory perception of smell"
}